{
  "gene": "UniProtKB:P46063",
  "term_id": "GO:0005737",
  "gene_symbol": "RECQL",
  "gene_name": "ATP-dependent DNA helicase Q1",
  "term_label": "cytoplasm"
}